otolith tethering [GO:0035889] (biological process) Relationships: is a type of multicellular organismal process [GO:0032501]; is part of otolith development [GO:0048840] References: PMID:14499652 Sources: GOC:dgh Definition: The attachment of a developing otolith to the kinocilia of tether cells in the inner ear.